histone H3R8me2 reader activity [GO:0140127] (molecular function) Note: Comment: Note that the residue position corresponds to the canonical human H3 histone (UniProtKB:P84243); this residue is conserved across all eukaryotes. Residue 1 is the first residue following removal of the initiating Methionine (Met). Note that each histone is encoded by multiple genes, and sequences may vary across different genes within an organism. Definition: A histone reader that recognizes a histone H3 dimethylate at arginine 8. The methylation can be symmetrical or asymmetrical. References: PMID:24589551 Relationships: is a type of histone H3 reader activity [GO:0140006]